tetracycline:proton antiporter activity [GO:0015520] (MF) Also known as: tetracyclin:hydrogen antiporter activity, tetracyclin:proton antiporter activity, tetracycline:hydrogen antiporter activity Sources: TC:2.A.1.2.4 Relationships: is a type of tetracycline transmembrane transporter activity [GO:0008493]; is a type of GO:0015078; is a type of GO:0015297 Definition: Enables the transfer of a solute or solutes from one side of a membrane to the other according to the reaction: H+(out) + tetracycline(in) = H+(in) + tetracycline(out).